heart process [GO:0003015] (biological process) Relationships: is a type of circulatory system process [GO:0003013] Also known as: cardiac process Subtypes: regulation of systemic arterial blood pressure by atrial baroreceptor feedback [GO:0002015], heart contraction [GO:0060047] Sources: GOC:mtg_cardio Definition: A circulatory system process carried out by the heart. The heart is a hollow, muscular organ, which, by contracting rhythmically, keeps up the circulation of the blood. The heart is a hollow, muscular organ, which, by contracting rhythmically, keeps up the circulation of the blood.